{
  "term_id": "GO:0000149",
  "term_label": "SNARE binding",
  "gene_symbol": "TNFAIP2",
  "gene": "UniProtKB:Q03169",
  "gene_name": "Tumor necrosis factor alpha-induced protein 2"
}